{
  "term_id": "GO:0006357",
  "term_label": "regulation of transcription by RNA polymerase II",
  "gene_symbol": "ZNF415",
  "gene_name": "Zinc finger protein 415",
  "gene": "UniProtKB:Q09FC8"
}